negative regulation of adenosine receptor signaling pathway [GO:0060169] (biological process) Definition: Any process that stops, prevents, or reduces the frequency, rate or extent of the adenosine receptor signaling pathway. The adenosine receptor pathway is the series of molecular signals generated as a consequence of an adenosine receptor binding to one of its physiological ligands. Relationships: is a type of negative regulation of G protein-coupled receptor signaling pathway [GO:0045744]; is a type of regulation of adenosine receptor signaling pathway [GO:0060167]; negatively regulates G protein-coupled adenosine receptor signaling pathway [GO:0001973] Sources: GOC:dph Also known as: negative regulation of adenosine receptor signalling pathway